{
  "term_label": "cytoplasm",
  "gene_name": "FYVE, RhoGEF and PH domain-containing protein 4",
  "gene": "UniProtKB:Q96M96",
  "gene_symbol": "FGD4",
  "term_id": "GO:0005737"
}